{
  "gene_name": "Collagen and calcium-binding EGF domain-containing protein 1",
  "gene": "UniProtKB:Q6UXH8",
  "term_id": "GO:0031012",
  "term_label": "extracellular matrix",
  "gene_symbol": "CCBE1"
}